brassinosteroid metabolic process [GO:0016131] (biological process) Definition: The chemical reactions and pathways involving brassinosteroids, any of a group of steroid derivatives that occur at very low concentrations in plant tissues and may have hormone-like effects. Sources: ISBN:0192801023 Also known as: brassinosteroid metabolism Relationships: is a type of steroid metabolic process [GO:0008202]; is a type of hormone metabolic process [GO:0042445] Subtypes: GO:0016132, GO:0016133